{
  "term_id": "GO:0005634",
  "term_label": "nucleus",
  "gene_symbol": "MAGEA9",
  "gene": "UniProtKB:P43362",
  "gene_name": "Melanoma-associated antigen 9"
}